{
  "term_id": "GO:0016477",
  "gene_symbol": "CD151",
  "gene": "UniProtKB:P48509",
  "term_label": "cell migration",
  "gene_name": "CD151 antigen"
}